{
  "gene_symbol": "RHEB",
  "gene_name": "GTP-binding protein Rheb",
  "term_label": "protein serine/threonine kinase activator activity",
  "term_id": "GO:0043539",
  "gene": "UniProtKB:Q15382"
}